ceramide glucosyltransferase activity [GO:0008120] (MF) Definition: Catalysis of the reaction: an N-acylsphing-4-enine + UDP-alpha-D-glucose = a beta-D-glucosyl-(1<->1')-N-acylsphing-4-enine + H+ + UDP. Sources: RHEA:12088 Also known as: UDP-glucose-ceramide glucosyltransferase activity, UDP-glucose:N-acylsphingosine D-glucosyltransferase activity, UDP-glucose:ceramide glucosyltransferase activity, UDPglucose:N-acylsphingosine D-glucosyltransferase activity, ceramide:UDP-glucose glucosyltransferase activity, ceramide:UDPGlc glucosyltransferase activity, glucosylceramide synthase activity, uridine diphosphoglucose-ceramide glucosyltransferase activity Relationships: is a type of GO:0035251